{
  "gene_symbol": "TNRC18",
  "term_id": "UNKNOWN:0002",
  "gene_name": "Trinucleotide repeat-containing gene 18 protein",
  "gene": "UniProtKB:O15417",
  "term_label": "Unknown biological process"
}